symbiont-mediated suppression of host translation elongation [GO:0141155] (biological process) Relationships: is a type of symbiont-mediated perturbation of host gene expression [GO:0039656] Definition: A process in which a symbiont inhibits or disrupts the translation elongation of host mRNA into protein, for example by directly inhibiting elongation factors. The host is defined as the larger of the organisms involved in a symbiotic interaction. References: PMID:10657208, PMID:18281405, PMID:18448518